{
  "gene_symbol": "UMOD",
  "term_id": "GO:1990266",
  "gene": "UniProtKB:P07911",
  "gene_name": "Uromodulin",
  "term_label": "neutrophil migration"
}